viral budding from outer nuclear membrane [GO:0046772] (biological process) Relationships: is a type of GO:0046765 Definition: The envelopment of a virus, in which the naked capsid evaginates from the host outer nuclear membrane system, thus acquiring a membrane envelope. Also known as: virus budding from outer nuclear membrane by viral capsid envelopment, outer nuclear membrane viral budding during viral capsid envelopment, viral budding from outer nuclear membrane during viral capsid envelopment, virus budding from outer nuclear membrane during viral capsid envelopment Sources: ISBN:0072370319